positive regulation of blood microparticle formation [GO:2000334] (biological process) Also known as: positive regulation of microparticle generation, positive regulation of microparticle release Subtypes: positive regulation of endothelial microparticle formation [GO:2000337] Sources: GOC:BHF, GOC:mah Relationships: is_a GO:0051094; is a type of GO:0051130; is a type of GO:2000332; positively regulates blood microparticle formation [GO:0072564] Definition: Any process that activates or increases the frequency, rate or extent of blood microparticle formation.